intraciliary transport involved in cilium assembly [GO:0035735] (biological process) Relationships: is a type of intraciliary transport [GO:0042073]; is part of cilium assembly [GO:0060271] Definition: The bidirectional movement of large protein complexes along microtubules within a cilium that contributes to cilium assembly. Also known as: intraflagellar transport, intraciliary transport involved in cilium morphogenesis, intraflagellar transport involved in cilium morphogenesis Sources: GOC:bf, GOC:cilia